T cell tolerance induction to tumor cell [GO:0002411] (biological process) Regulation: regulated by regulation of T cell tolerance induction to tumor cell [GO:0002846]; negatively regulated by negative regulation of T cell tolerance induction to tumor cell [GO:0002847]; positively regulated by GO:0002848 Definition: A process of tolerance induction dependent on T cells which leads to immunological tolerance of a tumor. Relationships: is_a tolerance induction to tumor cell [GO:0002413]; is a type of T cell mediated immune response to tumor cell [GO:0002424]; is a type of peripheral T cell tolerance induction [GO:0002458] References: PMID:16730260 Sources: GOC:add, ISBN:0781735149